{
  "gene_symbol": "ZNF25",
  "gene_name": "Zinc finger protein 25",
  "term_id": "GO:0000977",
  "term_label": "RNA polymerase II transcription regulatory region sequence-specific DNA binding",
  "gene": "UniProtKB:P17030"
}